{
  "term_label": "positive regulation of type II interferon-mediated signaling pathway",
  "gene_name": "Protein mono-ADP-ribosyltransferase PARP9",
  "gene_symbol": "PARP9",
  "gene": "UniProtKB:Q8IXQ6",
  "term_id": "GO:0060335"
}